{
  "gene": "UniProtKB:Q8IZ40",
  "term_id": "GO:0006357",
  "term_label": "regulation of transcription by RNA polymerase II",
  "gene_name": "REST corepressor 2",
  "gene_symbol": "RCOR2"
}